{
  "gene_name": "Protein FAM170A",
  "gene_symbol": "FAM170A",
  "gene": "UniProtKB:A1A519",
  "term_id": "GO:0009566",
  "term_label": "fertilization"
}